{
  "term_label": "Golgi apparatus",
  "gene_symbol": "ZDHHC12",
  "gene": "UniProtKB:Q96GR4",
  "term_id": "GO:0005794",
  "gene_name": "Palmitoyltransferase ZDHHC12"
}